photosystem II stabilization [GO:0042549] (biological process) Definition: The stabilization of the photosystem II protein complex, resulting from the phosphorylation of its structural protein subunits, in a cell actively involved in photosynthesis. Sources: GOC:go_curators Relationships: is a type of GO:0042548